isoquinoline alkaloid metabolic process [GO:0033076] (BP) Subtypes: isoquinoline alkaloid biosynthetic process [GO:0033075], morphine metabolic process [GO:0071272], isoquinoline alkaloid catabolic process [GO:0071274], codeine metabolic process [GO:2001291] Definition: The chemical reactions and pathways involving isoquinoline alkaloids, alkaloid compounds that contain bicyclic N-containing aromatic rings and are derived from a 3,4-dihydroxytyramine (dopamine) precursor that undergoes a Schiff base addition with aldehydes of different origin. References: PMID:26503307 Sources: GOC:mah Also known as: isoquinoline alkaloid metabolism, ipecac alkaloid metabolism Relationships: is a type of alkaloid metabolic process [GO:0009820]